{
  "term_label": "Unknown cellular component",
  "term_id": "UNKNOWN:0003",
  "gene_symbol": "DHX29",
  "gene": "UniProtKB:Q7Z478",
  "gene_name": "ATP-dependent RNA helicase DHX29"
}